{
  "term_id": "GO:0140517",
  "term_label": "protein-RNA adaptor activity",
  "gene_symbol": "SH3BGRL",
  "gene": "UniProtKB:O75368",
  "gene_name": "Adapter SH3BGRL"
}